symmetric synapse [GO:0032280] (cellular component) Note: The term 'symmetric' in this name refers only to gross morphology. There is no implication of functional symmetry. Subtypes: GO:0098983 Also known as: Gray's type II synapse Relationships: is a type of neuron to neuron synapse [GO:0098984] Definition: A synapse that lacks an electron dense postsynaptic specialization. In vertebtrates, these occur primarily on dendrite shafts and neuronal cell bodies and involve persynapses containing clusters of predominantly flattened or elongated vesicles and are typically inhibitory. Sources: GOC:dgh, GOC:ef